short-chain fatty acid transmembrane transport [GO:0015913] (biological process) Definition: The directed movement of short-chain fatty acids into a cell or organelle. A short-chain fatty acid has an aliphatic tail containing fewer than 6 carbons. Sources: GOC:ai Also known as: short-chain fatty acid uptake, short-chain fatty acid import Note: While there is not universal consensus on the lengths of short-, medium-, long- and very-long-chain fatty acids, the GO uses the definitions in ChEBI (see CHEBI:26666, CHEBI:59554, CHEBI:15904 and CHEBI:27283). Relationships: is_a short-chain fatty acid transport [GO:0015912]; is a type of fatty acid transmembrane transport [GO:1902001] Subtypes: propanoate transmembrane transport [GO:0015730]